{
  "term_id": "GO:0016020",
  "gene_name": "Myotubularin-related protein 10",
  "gene": "UniProtKB:Q9NXD2",
  "term_label": "membrane",
  "gene_symbol": "MTMR10"
}